positive regulation of mitochondrial ATP synthesis coupled electron transport [GO:1905448] (biological process) Relationships: is a type of positive regulation of metabolic process [GO:0009893]; is a type of regulation of mitochondrial ATP synthesis coupled electron transport [GO:1905446]; positively regulates mitochondrial ATP synthesis coupled electron transport [GO:0042775] Definition: Any process that activates or increases the frequency, rate or extent of mitochondrial ATP synthesis coupled electron transport. Also known as: up regulation of mitochondrial ATP synthesis coupled electron transport, up-regulation of mitochondrial ATP synthesis coupled electron transport, upregulation of mitochondrial ATP synthesis coupled electron transport, activation of mitochondrial ATP synthesis coupled electron transport References: PMID:23707074 Sources: GOC:PARL, GOC:TermGenie, GOC:bc, GO_REF:0000058